{
  "gene_name": "Zinc finger SWIM domain-containing protein 6",
  "gene_symbol": "ZSWIM6",
  "gene": "UniProtKB:Q9HCJ5",
  "term_id": "UNKNOWN:0001",
  "term_label": "Unknown molecular function"
}